positive regulation of epithelial cell-cell adhesion involved in epithelium migration [GO:1903683] (biological process) Also known as: up regulation of epithelial cell-cell adhesion involved in epithelium migration, up-regulation of epithelial cell-cell adhesion involved in epithelium migration, upregulation of epithelial cell-cell adhesion involved in epithelium migration, activation of epithelial cell-cell adhesion involved in epithelium migration References: PMID:18394891 Sources: GOC:TermGenie, GOC:als, GO_REF:0000058 Relationships: is_a positive regulation of cell-cell adhesion [GO:0022409]; is_a positive regulation of multicellular organismal process [GO:0051240]; is a type of regulation of epithelial cell-cell adhesion involved in epithelium migration [GO:1903681]; positively regulates GO:0090137 Definition: Any process that activates or increases the frequency, rate or extent of epithelial cell-cell adhesion involved in epithelium migration.